{
  "gene_symbol": "ZNF417",
  "term_label": "nucleus",
  "gene_name": "Zinc finger protein 417",
  "gene": "UniProtKB:Q8TAU3",
  "term_id": "GO:0005634"
}